response to interleukin-12 [GO:0070671] (biological process) Definition: Any process that results in a change in state or activity of a cell or an organism (in terms of movement, secretion, enzyme production, gene expression, etc.) as a result of an interleukin-12 stimulus. Subtypes: cellular response to interleukin-12 [GO:0071349] Sources: GOC:mah Relationships: is a type of response to cytokine [GO:0034097] Also known as: response to IL-12